6-O-methyl-deacetylisoipecoside beta-glucosidase activity [GO:0102413] (molecular function) Definition: Catalysis of the reaction: 6-O-methyl-N-deacetylisoipecoside + H2O = 6-O-methyl-N-deacetylisoipecoside aglycon + D-glucose. Sources: RHEA:78891 Relationships: is a type of hydrolase activity, hydrolyzing O-glycosyl compounds [GO:0004553]